{
  "term_label": "vesicle membrane",
  "term_id": "GO:0012506",
  "gene_symbol": "ANXA3",
  "gene_name": "Annexin A3",
  "gene": "UniProtKB:P12429"
}